positive regulation of myeloid dendritic cell chemotaxis [GO:2000529] (biological process) Relationships: is a type of positive regulation of dendritic cell chemotaxis [GO:2000510]; is a type of regulation of myeloid dendritic cell chemotaxis [GO:2000527]; positively regulates myeloid dendritic cell chemotaxis [GO:0002408] Definition: Any process that activates or increases the frequency, rate or extent of myeloid dendritic cell chemotaxis. Sources: GOC:obol